telencephalon microglial cell migration [GO:0022033] (biological process) Sources: GOC:cls, GOC:dgh, GOC:dph, GOC:jid, GO_REF:0000021 Relationships: is a type of telencephalon glial cell migration [GO:0022030] Definition: The orderly movement of microglial cells through the telencephalon.